positive regulation of heat dissipation [GO:0031656] (biological process) Sources: GOC:dph, GOC:mah, GOC:tb Relationships: is a type of regulation of heat dissipation [GO:0031654]; is a type of positive regulation of multicellular organismal process [GO:0051240]; positively regulates GO:0031653 Also known as: up regulation of heat dissipation, up-regulation of heat dissipation, upregulation of heat dissipation, activation of heat dissipation, stimulation of heat dissipation Definition: Any process that activates or increases the rate or extent of heat dissipation.